{
  "term_id": "GO:0004301",
  "gene": "UniProtKB:P07099",
  "gene_symbol": "EPHX1",
  "term_label": "epoxide hydrolase activity",
  "gene_name": "Epoxide hydrolase 1"
}